larval burrowing behavior [GO:0035181] (biological process) References: PMID:12848927, PMID:12848939 Also known as: larval burrowing behaviour Relationships: is a type of larval locomotory behavior [GO:0008345] Definition: Digging into the substrate by non-feeding larvae in search for food-free sites suitable for pupation.